{
  "term_id": "GO:0007413",
  "term_label": "axonal fasciculation",
  "gene": "UniProtKB:Q9NQ79",
  "gene_name": "Cartilage acidic protein 1",
  "gene_symbol": "CRTAC1"
}